{
  "gene_symbol": "TARS2",
  "term_label": "threonyl-tRNA aminoacylation",
  "gene": "UniProtKB:Q9BW92",
  "term_id": "GO:0006435",
  "gene_name": "Threonine--tRNA ligase, mitochondrial"
}